reproductive fruiting body development [GO:0030582] (biological process) Definition: The process whose specific outcome is the progression of a reproductive fruiting body over time, from its formation to the mature structure. A reproductive fruiting body is a multicellular reproductive structure that contains spores. Subtypes: sporocarp development [GO:0030584], aecium development [GO:0075267], GO:0120165, protoperithecium formation [GO:0120166] Note: This term describes the development of a fruiting body that is a spore-bearing organ. It is not intended to describe the development of myxococcal fruiting bodies. Regulation: regulated by regulation of reproductive fruiting body development [GO:0031155] Sources: GOC:mah, GOC:mtg_sensu Also known as: fruiting body formation Relationships: is a type of spore-bearing structure development [GO:0075259]